{
  "term_label": "sarcolemma",
  "gene": "UniProtKB:Q99828",
  "term_id": "GO:0042383",
  "gene_name": "Calcium and integrin-binding protein 1",
  "gene_symbol": "CIB1"
}